{
  "gene_name": "DCN1-like protein 1",
  "gene": "UniProtKB:Q96GG9",
  "gene_symbol": "DCUN1D1",
  "term_label": "ubiquitin-like protein binding",
  "term_id": "GO:0032182"
}